{
  "gene_name": "ADP-ribosylation factor-like protein 3",
  "gene": "UniProtKB:P36405",
  "term_label": "microtubule cytoskeleton",
  "gene_symbol": "ARL3",
  "term_id": "GO:0015630"
}